{
  "term_label": "plasma membrane",
  "gene_symbol": "PRMT8",
  "term_id": "GO:0005886",
  "gene": "UniProtKB:Q9NR22",
  "gene_name": "Protein arginine N-methyltransferase 8"
}